{
  "term_label": "cell surface receptor signaling pathway",
  "term_id": "GO:0007166",
  "gene_name": "T cell receptor beta variable 30",
  "gene_symbol": "TRBV30",
  "gene": "UniProtKB:A0A0K0K1B3"
}